nucleotide-excision repair factor 3 complex [GO:0000112] (CC) Relationships: is a type of nucleotide-excision repair complex [GO:0000109]; has part transcription factor TFIIH core complex [GO:0000439] References: PMID:10915862, PMID:14500720, PMID:7813015 Sources: GOC:ew Definition: One of several protein complexes involved in nucleotide-excision repair; possesses endodeoxynuclease and DNA helicase activities. In S. cerevisiae, it is composed of Rad2p and the core TFIIH-Ssl2p complex (core TFIIH is composed of Rad3p, Tfb1p, Tfb2p, Ssl1p, Tfb4p and Tfb5p. Note that Ssl2p is also called Rad25p). Also known as: NEF3 complex Note: Note that process and function information are included in the term and definition for the purpose of describing and distinguishing the complex.